primary alcohol metabolic process [GO:0034308] (biological process) Subtypes: ethanol metabolic process [GO:0006067], octanol metabolic process [GO:0006070], GO:0006580, GO:0006772, GO:0009441, methanol metabolic process [GO:0015945], farnesol metabolic process [GO:0016487], GO:0032341, phytol metabolic process [GO:0033306], primary alcohol biosynthetic process [GO:0034309], primary alcohol catabolic process [GO:0034310], cortisol metabolic process [GO:0034650], retinol metabolic process [GO:0042572], GO:0044598, glycerol to glycerone phosphate metabolic process [GO:0061610], GO:0061720, GO:0070291, aromatic primary alcohol metabolic process [GO:1902654], glycine catabolic process to isobutanol [GO:1902696], L-valine catabolic process to isobutanol [GO:1902697] Relationships: is a type of GO:0006066 Sources: GOC:mah Definition: The chemical reactions and pathways involving primary alcohols. A primary alcohol is any alcohol in which a hydroxy group, -OH, is attached to a saturated carbon atom which has either three hydrogen atoms attached to it or only one other carbon atom and two hydrogen atoms attached to it. Also known as: monohydric alcohol metabolic process, primary alcohol metabolism